translation release factor activity [GO:0003747] (MF) Sources: ISBN:0198547684 Relationships: is_a translation termination factor activity [GO:0008079] Subtypes: translation release factor activity, codon specific [GO:0016149], translation release factor activity, codon nonspecific [GO:0016150] Definition: Involved in catalyzing the release of a nascent polypeptide chain from a ribosome.